{
  "term_label": "FANCM-MHF complex",
  "term_id": "GO:0071821",
  "gene": "UniProtKB:Q8N2Z9",
  "gene_symbol": "CENPS",
  "gene_name": "Centromere protein S"
}